{
  "term_id": "GO:0005049",
  "gene_symbol": "RANBP17",
  "gene": "UniProtKB:Q9H2T7",
  "gene_name": "Ran-binding protein 17",
  "term_label": "nuclear export signal receptor activity"
}